{
  "gene_name": "Vacuolar protein sorting-associated protein 45",
  "term_label": "Golgi membrane",
  "gene": "UniProtKB:Q9NRW7",
  "term_id": "GO:0000139",
  "gene_symbol": "VPS45"
}